{
  "gene_name": "Pyroglutamyl-peptidase 1-like protein",
  "term_id": "UNKNOWN:0002",
  "gene": "UniProtKB:A6NFU8",
  "gene_symbol": "PGPEP1L",
  "term_label": "Unknown biological process"
}